{
  "gene": "UniProtKB:Q9NUD7",
  "gene_symbol": "C20orf96",
  "term_id": "UNKNOWN:0003",
  "gene_name": "Uncharacterized protein C20orf96",
  "term_label": "Unknown cellular component"
}